{
  "gene_symbol": "CHODL",
  "gene_name": "Chondrolectin",
  "term_id": "GO:0005737",
  "term_label": "cytoplasm",
  "gene": "UniProtKB:Q9H9P2"
}